{
  "term_id": "UNKNOWN:0002",
  "gene_name": "Zinc finger BED domain-containing protein 4",
  "term_label": "Unknown biological process",
  "gene_symbol": "ZBED4",
  "gene": "UniProtKB:O75132"
}